{
  "gene_name": "Derlin-3",
  "gene_symbol": "DERL3",
  "term_label": "endoplasmic reticulum unfolded protein response",
  "term_id": "GO:0030968",
  "gene": "UniProtKB:Q96Q80"
}